phosphatidylinositol 3-kinase complex, class IB [GO:0005944] (cellular component) Also known as: 1-phosphatidylinositol-4-phosphate 3-kinase, class IB complex, class IB PI3K complex, phosphoinositide 3-kinase complex, class IB, 1-phosphatidylinositol-4-phosphate kinase, class IB complex References: PMID:9255069, PMID:9759495 Definition: A class I phosphatidylinositol 3-kinase complex that possesses 1-phosphatidylinositol-4-phosphate 3-kinase activity; comprises a catalytic class IB phosphoinositide 3-kinase (PI3K) subunit and an associated regulatory subunit that is larger than, and unrelated to, the p85 proteins present in class IA complexes. Class IB PI3Ks are stimulated by G-proteins and do not interact with the SH2-domain containing adaptors that bind to Class IA PI3Ks. Relationships: is a type of phosphatidylinositol 3-kinase complex, class I [GO:0097651]